negative regulation of renal sodium excretion [GO:0035814] (biological process) Sources: GOC:mtg_25march11, GOC:yaf Relationships: is a type of regulation of renal sodium excretion [GO:0035813]; is a type of negative regulation of secretion [GO:0051048]; is a type of negative regulation of multicellular organismal process [GO:0051241]; negatively regulates GO:0035812 Note: The amount of sodium excreted in urine over a unit of time can be decreased by decreasing the volume of urine produced (antidiuresis) and/or by decreasing the concentration of sodium in the urine. Definition: Any process that decreases the amount of sodium excreted in urine over a unit of time. Subtypes: negative regulation of renal sodium excretion by angiotensin [GO:0035820]